detection of osmotic stimulus [GO:0043575] (biological process) Definition: The series of events in which a stimulus indicating an increase or decrease in the concentration of solutes outside the organism or cell is received and converted into a molecular signal. Sources: GOC:jl Relationships: is a type of response to osmotic stress [GO:0006970]; is a type of detection of abiotic stimulus [GO:0009582]